{
  "gene_symbol": "NCSTN",
  "term_id": "UNKNOWN:0001",
  "term_label": "Unknown molecular function",
  "gene_name": "Nicastrin",
  "gene": "UniProtKB:Q92542"
}